{
  "term_label": "cytoplasm",
  "gene_symbol": "AGFG1",
  "term_id": "GO:0005737",
  "gene_name": "Arf-GAP domain and FG repeat-containing protein 1",
  "gene": "UniProtKB:P52594"
}